regulation of extent of cell growth [GO:0061387] (biological process) Definition: Any process that modulates the extent of cell growth. Sources: GOC:mah, GOC:vw Relationships: is a type of regulation of cell growth [GO:0001558]; is part of GO:0008361 Subtypes: GO:0030516, GO:0048670, regulation of sprouting of injured axon [GO:0048686]